{
  "term_id": "UNKNOWN:0001",
  "term_label": "Unknown molecular function",
  "gene_symbol": "POLR1F",
  "gene": "UniProtKB:Q3B726",
  "gene_name": "DNA-directed RNA polymerase I subunit RPA43"
}